positive regulation of protein-pyridoxal-5-phosphate linkage [GO:1904287] (biological process) Relationships: is a type of positive regulation of protein modification process [GO:0031401]; is a type of regulation of protein-pyridoxal-5-phosphate linkage [GO:1904285]; positively regulates protein-pyridoxal-5-phosphate linkage [GO:0018352] Also known as: stimulation of protein-pyridoxal-5-phosphate linkage, up regulation of protein-pyridoxal-5-phosphate linkage, up-regulation of protein-pyridoxal-5-phosphate linkage, upregulation of protein-pyridoxal-5-phosphate linkage, activation of protein-pyridoxal-5-phosphate linkage Definition: Any process that activates or increases the frequency, rate or extent of protein-pyridoxal-5-phosphate linkage. References: PMID:25957689 Sources: GOC:TermGenie, GO_REF:0000058